{
  "gene_name": "eIF5-mimic protein 1",
  "term_label": "Unknown biological process",
  "term_id": "UNKNOWN:0002",
  "gene": "UniProtKB:Q9Y6E2",
  "gene_symbol": "BZW2"
}